negative regulation of glycoprotein metabolic process [GO:1903019] (biological process) Subtypes: negative regulation of glycoprotein biosynthetic process [GO:0010561], negative regulation by host of viral glycoprotein metabolic process [GO:0044871], negative regulation of elastin catabolic process [GO:0060311] Relationships: is a type of GO:0051248; is a type of GO:1903018; negatively regulates glycoprotein metabolic process [GO:0009100] Definition: Any process that stops, prevents or reduces the frequency, rate or extent of glycoprotein metabolic process. References: PMID:23544079 Sources: GOC:BHF, GOC:TermGenie, GOC:rl, GO_REF:0000058 Also known as: down regulation of glycoprotein metabolic process, down regulation of glycoprotein metabolism, down-regulation of glycoprotein metabolic process, down-regulation of glycoprotein metabolism, downregulation of glycoprotein metabolic process, downregulation of glycoprotein metabolism, negative regulation of glycoprotein metabolism, inhibition of glycoprotein metabolic process, inhibition of glycoprotein metabolism Note: human serum amyloid P component (SAP) P02743 inhibits viral neuraminidase, NA (exo-alpha-sialidase activity) and thus the metabolism of glycoproteins, demonstrated in Figure 4A PMID:23544079, (IDA), the negative regulation term would be applied to this protein